{
  "term_id": "UNKNOWN:0001",
  "gene_name": "Basement membrane-specific heparan sulfate proteoglycan core protein",
  "term_label": "Unknown molecular function",
  "gene_symbol": "HSPG2",
  "gene": "UniProtKB:P98160"
}